{
  "gene_name": "DNA helicase MCM9",
  "gene_symbol": "MCM9",
  "term_id": "GO:0042555",
  "term_label": "MCM complex",
  "gene": "UniProtKB:Q9NXL9"
}